{
  "term_id": "GO:0045202",
  "gene_name": "Muscarinic acetylcholine receptor M4",
  "gene_symbol": "CHRM4",
  "term_label": "synapse",
  "gene": "UniProtKB:P08173"
}